{
  "term_label": "Unknown biological process",
  "gene_name": "Cilia- and flagella-associated protein 144",
  "gene_symbol": "CFAP144",
  "gene": "UniProtKB:A6NL82",
  "term_id": "UNKNOWN:0002"
}